{
  "gene_name": "Ski-like protein",
  "term_id": "GO:0000978",
  "gene_symbol": "SKIL",
  "term_label": "RNA polymerase II cis-regulatory region sequence-specific DNA binding",
  "gene": "UniProtKB:P12757"
}